{
  "gene": "UniProtKB:Q15059",
  "gene_symbol": "BRD3",
  "term_id": "GO:0006338",
  "gene_name": "Bromodomain-containing protein 3",
  "term_label": "chromatin remodeling"
}